{
  "gene_symbol": "STIMATE",
  "term_id": "GO:0005246",
  "gene_name": "Store-operated calcium entry regulator STIMATE",
  "gene": "UniProtKB:Q86TL2",
  "term_label": "calcium channel regulator activity"
}